L-arabinose biosynthetic process [GO:0033357] (biological process) Sources: GOC:mah Definition: The chemical reactions and pathways resulting in the formation of L-arabinose, arabino-pentose. Relationships: is_a arabinose biosynthetic process [GO:0019567]; is a type of L-arabinose metabolic process [GO:0046373] Also known as: L-arabinose anabolism, L-arabinose biosynthesis, L-arabinose formation, L-arabinose synthesis